{
  "gene_name": "Tumor necrosis factor receptor superfamily member 5",
  "gene": "UniProtKB:P25942",
  "term_id": "GO:0042113",
  "gene_symbol": "CD40",
  "term_label": "B cell activation"
}